{
  "gene": "UniProtKB:Q8N4V2",
  "gene_symbol": "SVOP",
  "term_label": "Unknown biological process",
  "gene_name": "Synaptic vesicle 2-related protein",
  "term_id": "UNKNOWN:0002"
}